{
  "gene_symbol": "SLC38A7",
  "gene": "UniProtKB:Q9NVC3",
  "term_id": "GO:0016020",
  "gene_name": "Sodium-coupled neutral amino acid transporter 7",
  "term_label": "membrane"
}